positive regulation of oskar mRNA translation [GO:0046012] (biological process) Definition: Any process that activates or increases the frequency, rate or extent of oskar mRNA translation. Sources: GOC:go_curators Also known as: up regulation of oskar mRNA translation, up-regulation of oskar mRNA translation, upregulation of oskar mRNA translation, activation of oskar mRNA translation, stimulation of oskar mRNA translation Relationships: is a type of positive regulation of translation [GO:0045727]; is a type of regulation of oskar mRNA translation [GO:0046011]